L-valine biosynthetic process [GO:0009099] (biological process) Also known as: valine anabolism, valine biosynthesis, valine formation, valine synthesis Sources: GOC:ai Definition: The chemical reactions and pathways resulting in the formation of valine, 2-amino-3-methylbutanoic acid. Relationships: is a type of valine metabolic process [GO:0006573]; is a type of pyruvate family amino acid biosynthetic process [GO:0009079]; is a type of branched-chain amino acid biosynthetic process [GO:0009082]; has part GO:0003984; BFO_0000051 dihydroxy-acid dehydratase activity [GO:0004160]; has part GO:0004455; has part L-valine-2-oxoglutarate transaminase activity [GO:0052655]